{
  "gene_symbol": "OTUD7B",
  "term_label": "cysteine-type deubiquitinase activity",
  "gene_name": "OTU domain-containing protein 7B",
  "term_id": "GO:0004843",
  "gene": "UniProtKB:Q6GQQ9"
}